{
  "term_id": "GO:0007224",
  "gene": "UniProtKB:Q96F81",
  "term_label": "smoothened signaling pathway",
  "gene_name": "Protein dispatched homolog 1",
  "gene_symbol": "DISP1"
}